{
  "gene_symbol": "PPP1R15A",
  "gene_name": "Protein phosphatase 1 regulatory subunit 15A",
  "gene": "UniProtKB:O75807",
  "term_label": "response to endoplasmic reticulum stress",
  "term_id": "GO:0034976"
}